{
  "gene": "UniProtKB:Q99466",
  "term_id": "UNKNOWN:0003",
  "gene_symbol": "NOTCH4",
  "gene_name": "Neurogenic locus notch homolog protein 4",
  "term_label": "Unknown cellular component"
}